{
  "term_id": "GO:0030020",
  "gene_symbol": "COL4A4",
  "gene": "UniProtKB:P53420",
  "term_label": "extracellular matrix structural constituent conferring tensile strength",
  "gene_name": "Collagen alpha-4(IV) chain"
}